{
  "term_id": "GO:0005615",
  "term_label": "extracellular space",
  "gene_name": "Zinc-alpha-2-glycoprotein",
  "gene": "UniProtKB:P25311",
  "gene_symbol": "AZGP1"
}